{
  "term_label": "RNA polymerase II cis-regulatory region sequence-specific DNA binding",
  "gene_name": "Upstream stimulatory factor 2",
  "term_id": "GO:0000978",
  "gene_symbol": "USF2",
  "gene": "UniProtKB:Q15853"
}